{
  "term_label": "Unknown biological process",
  "gene_name": "Tyrosine--tRNA ligase, cytoplasmic",
  "gene_symbol": "YARS1",
  "term_id": "UNKNOWN:0002",
  "gene": "UniProtKB:P54577"
}